{
  "gene_symbol": "SEPTIN10",
  "gene": "UniProtKB:Q9P0V9",
  "term_id": "GO:0015630",
  "term_label": "microtubule cytoskeleton",
  "gene_name": "Septin-10"
}